{
  "gene_name": "Large ribosomal subunit protein uL10m",
  "term_label": "structural constituent of ribosome",
  "gene_symbol": "MRPL10",
  "term_id": "GO:0003735",
  "gene": "UniProtKB:Q7Z7H8"
}